retrograde dendritic transport [GO:0098934] (biological process) Definition: The directed movement of organelles or molecules along microtubules in a dendrite from the postsynapse towards the cell body. Sources: GOC:dos Relationships: is a type of dendritic transport [GO:0098935]; occurs in dendrite cytoplasm [GO:0032839]